{
  "gene": "UniProtKB:Q9Y2I9",
  "gene_name": "TBC1 domain family member 30",
  "term_label": "Unknown biological process",
  "term_id": "UNKNOWN:0002",
  "gene_symbol": "TBC1D30"
}